{
  "gene": "UniProtKB:Q9Y303",
  "gene_symbol": "AMDHD2",
  "term_id": "GO:0006046",
  "gene_name": "N-acetylglucosamine-6-phosphate deacetylase",
  "term_label": "N-acetylglucosamine catabolic process"
}